{
  "term_label": "actin filament binding",
  "gene": "UniProtKB:Q12965",
  "term_id": "GO:0051015",
  "gene_name": "Unconventional myosin-Ie",
  "gene_symbol": "MYO1E"
}